regulation of chlorophyll biosynthetic process [GO:0010380] (biological process) Relationships: is a type of regulation of chlorophyll metabolic process [GO:0090056]; is a type of regulation of tetrapyrrole biosynthetic process [GO:1901463]; regulates chlorophyll biosynthetic process [GO:0015995] Subtypes: GO:1902325, positive regulation of chlorophyll biosynthetic process [GO:1902326] References: PMID:17291312 Definition: Any process that modulates the frequency, rate or extent of the chemical reactions and pathways resulting in the formation of chlorophyll, any compound of magnesium complexed in a porphyrin (tetrapyrrole) ring and which functions as a photosynthetic pigment, from less complex precursors.